glycolytic process from fructose through fructose-6-phosphate [GO:0061616] (biological process) Sources: GOC:dph, ISBN:0201090910, ISBN:0879010479 Definition: The glycolytic process through fructose-6-phosphate in which fructose is catabolized into pyruvate. Relationships: is a type of fructose catabolic process [GO:0006001]; is_a GO:0061615; has part GO:0008865 Also known as: glycolysis from fructose through fructose-6-phosphate